{
  "term_label": "regulation of Notch signaling pathway",
  "gene_symbol": "LFNG",
  "term_id": "GO:0008593",
  "gene_name": "Beta-1,3-N-acetylglucosaminyltransferase lunatic fringe",
  "gene": "UniProtKB:Q8NES3"
}